monoacylglycerol biosynthetic process [GO:0006640] (biological process) Definition: The chemical reactions and pathways resulting in the formation of monoacylglycerol, any ester of glycerol in which any one of its hydroxyl groups has been acylated with a fatty acid, the other being non-esterified. Also known as: monoacylglycerol anabolism, monoacylglycerol biosynthesis, monoacylglycerol formation, monoacylglycerol synthesis, monoglyceride biosynthesis, monoglyceride biosynthetic process Sources: ISBN:0198506732 Relationships: is a type of monoacylglycerol metabolic process [GO:0046462]; is a type of GO:0046463